{
  "term_label": "ribonucleoprotein complex",
  "gene": "UniProtKB:Q96DU9",
  "term_id": "GO:1990904",
  "gene_symbol": "PABPC5",
  "gene_name": "Polyadenylate-binding protein 5"
}